regulation of entry into reproductive diapause [GO:0061963] (biological process) Subtypes: negative regulation of entry into reproductive diapause [GO:0061964], positive regulation of entry into reproductive diapause [GO:0061965] References: PMID:27689881 Sources: GOC:ha Definition: Any process that modulates the rate or extent of the dormancy process that results in entry into reproductive diapause. Reproductive diapause is a form of diapause where the organism itself will remain fully active, including feeding and other routine activities, but the reproductive organs experience a tissue-specific reduction in metabolism, with characteristic triggering and releasing stimuli. Relationships: is a type of regulation of developmental process [GO:0050793]; regulates entry into reproductive diapause [GO:0055116]